{
  "term_label": "cell fate commitment",
  "gene_symbol": "WNT10A",
  "gene": "UniProtKB:Q9GZT5",
  "gene_name": "Protein Wnt-10a",
  "term_id": "GO:0045165"
}